regulation of lens epithelial cell proliferation [GO:2001109] (biological process) Subtypes: GO:2001110, positive regulation of lens epithelial cell proliferation [GO:2001111] Definition: Any process that modulates the frequency, rate or extent of lens epithelial cell proliferation. Sources: GOC:obol Relationships: is a type of regulation of epithelial cell proliferation [GO:0050678]; regulates lens epithelial cell proliferation [GO:0097166]